acetyl-coenzyme A:acetyl alcohol acetyltransferase activity [GO:0102720] (molecular function) Sources: EC:2.3.1.224 Definition: Catalysis of the reaction: acetyl-CoA + benzyl alcohol = benzyl acetate + CoA. Also converts (E)-cinnamyl alcohol into (E)-cinnamyl acetate. Relationships: is a type of GO:0016747